{
  "term_label": "morphogenesis of an epithelium",
  "gene_name": "Keratin, type I cytoskeletal 23",
  "gene_symbol": "KRT23",
  "term_id": "GO:0002009",
  "gene": "UniProtKB:Q9C075"
}